ribosomal skipping [GO:0075524] (biological process) Note: This term is intended to annotate gene products involved in the process of ribosomal skipping, not viral proteins produced by this translation process. Relationships: is a type of viral process [GO:0016032]; is part of viral translation [GO:0019081] Definition: A translation process in which a specific viral peptide prevents the ribosome from covalently linking a new inserted amino acid, and lets it continue translation, thereby cleaving the nascent protein while allowing translation to continue. Sources: GOC:bf, GOC:ch, GOC:jl, VZ:914